2'-hydroxyisoflavone reductase activity [GO:0047526] (molecular function) Relationships: is_a GO:0016628 Sources: RHEA:22560 Definition: Catalysis of the reaction: vestitone + NADP+ = 2'-hydroxyformononetin + NADPH + H+. Also known as: 2',7-dihydroxy-4',5'-methylenedioxyisoflavone reductase activity, NADPH:2'-hydroxyisoflavone oxidoreductase activity, isoflavone reductase activity, vestitone:NADP+ oxidoreductase activity